myosin II filament [GO:0097513] (cellular component) Relationships: is a type of myosin filament [GO:0032982] Sources: GOC:cjm, GOC:mah Definition: A bipolar filament composed of myosin II molecules.